GDP-fucose import into endoplasmic reticulum lumen [GO:0036084] (biological process) Definition: The directed movement of GDP-fucose into the endoplasmic reticulum lumen. GDP-fucose is a substance composed of fucose in glycosidic linkage with guanosine diphosphate. Relationships: is a type of GDP-fucose transmembrane transport [GO:0015783]; is a type of GO:0046967 Also known as: GDP-fucose import into endoplasmic reticulum, GDP-fucose transport across endoplasmic reticulum membrane, GDP-fucose transport into endoplasmic reticulum lumen References: PMID:3458237 Sources: GOC:sart